{
  "gene": "UniProtKB:Q6AI14",
  "gene_name": "Sodium_hydrogen exchanger 4",
  "term_id": "GO:0098719",
  "gene_symbol": "SLC9A4",
  "term_label": "sodium ion import across plasma membrane"
}